selenomethionine adenosyltransferase activity [GO:0098601] (molecular function) Relationships: is a type of GO:0016765 References: PMID:2339986 Sources: RHEA:31211 Definition: Catalysis of the reaction: L-selenomethionine + ATP + H2O = L-adenosylselenomethionine + phosphate + diphosphate.